glucoside 3-dehydrogenase activity [GO:0033757] (molecular function) Sources: EC:1.1.99.13 Definition: Catalysis of the reaction: sucrose + acceptor = 3-dehydro-alpha-D-glucosyl-beta-D-fructofuranoside + reduced acceptor. Also known as: D-aldohexopyranoside dehydrogenase, D-aldohexoside:(acceptor) 3-oxidoreductase, D-aldohexoside:acceptor 3-oxidoreductase, D-aldohexoside:cytochrome c oxidoreductase, hexopyranoside-cytochrome c oxidoreductase Relationships: is a type of GO:0016614